{
  "gene": "UniProtKB:Q6NSW7",
  "gene_name": "Homeobox protein NANOGP8",
  "gene_symbol": "NANOGP8",
  "term_id": "GO:0006357",
  "term_label": "regulation of transcription by RNA polymerase II"
}